{
  "gene_name": "Protein reprimo",
  "term_id": "GO:0007346",
  "term_label": "regulation of mitotic cell cycle",
  "gene": "UniProtKB:Q9NS64",
  "gene_symbol": "RPRM"
}